{
  "term_id": "GO:0005634",
  "gene": "UniProtKB:Q5FWF6",
  "gene_symbol": "ZNF789",
  "term_label": "nucleus",
  "gene_name": "Zinc finger protein 789"
}